potassium ion export across plasma membrane [GO:0097623] (biological process) Regulation: regulated by GO:1903764; negatively regulated by negative regulation of potassium ion export across plasma membrane [GO:1903765]; positively regulated by positive regulation of potassium ion export across plasma membrane [GO:1903766] Also known as: potassium export, potassium ion export, potassium export across plasma membrane, potassium ion export from cell References: PMID:11932440 Sources: GOC:vw Relationships: is a type of potassium ion transmembrane transport [GO:0071805]; is a type of export across plasma membrane [GO:0140115] Definition: The directed movement of potassium ions from inside of a cell, across the plasma membrane and into the extracellular region.